CMP salvage [GO:0006238] (biological process) Definition: Any process that generates CMP, cytidine monophosphate, from derivatives of it without de novo synthesis. Relationships: is a type of CMP biosynthetic process [GO:0009224]; is a type of GO:0010138 Also known as: cytidine monophosphate salvage Sources: GOC:jl